{
  "gene_name": "Kinesin-like protein KIF6",
  "gene": "UniProtKB:Q6ZMV9",
  "gene_symbol": "KIF6",
  "term_label": "ATP hydrolysis activity",
  "term_id": "GO:0016887"
}